{
  "term_label": "Unknown cellular component",
  "term_id": "UNKNOWN:0003",
  "gene": "UniProtKB:A0A0A0MT92",
  "gene_symbol": "IGLJ7",
  "gene_name": "Immunoglobulin lambda joining 7 (Fragment)"
}